{
  "gene_symbol": "CLEC4M",
  "term_id": "GO:0005537",
  "term_label": "D-mannose binding",
  "gene": "UniProtKB:Q9H2X3",
  "gene_name": "C-type lectin domain family 4 member M"
}